regulation of nucleotide-binding oligomerization domain containing 2 signaling pathway [GO:0070432] (biological process) Sources: GOC:add Also known as: regulation of NOD2 signaling pathway, regulation of nucleotide-binding oligomerization domain containing 2 signalling pathway Relationships: is a type of regulation of nucleotide-binding domain, leucine rich repeat containing receptor signaling pathway [GO:0070424]; regulates GO:0070431 Subtypes: negative regulation of nucleotide-binding oligomerization domain containing 2 signaling pathway [GO:0070433], positive regulation of nucleotide-binding oligomerization domain containing 2 signaling pathway [GO:0070434] Definition: Any process that modulates the frequency, rate, or extent of the nucleotide-binding oligomerization domain containing 2 (NOD2) pathway.